succinyl-CoA pathway [GO:0006781] (biological process) Definition: The chemical reactions that utilize succinyl-CoA in the synthesis of protoporphyrin IX. Relationships: is a type of succinyl-CoA metabolic process [GO:0006104]; is a type of porphyrin-containing compound biosynthetic process [GO:0006779]; is part of GO:0006780 Also known as: biosynthesis of protoporphyrin IX via succinyl CoA, biosynthesis of protoporphyrin IX via succinyl-CoA, biosynthetic process of protoporphyrin IX via succinyl CoA, biosynthetic process of protoporphyrin IX via succinyl-CoA, succinyl CoA pathway Sources: GOC:isa_complete, ISBN:0879010479